negative regulation of mitotic DNA replication initiation [GO:1903467] (biological process) Definition: Any process that stops, prevents or reduces the frequency, rate or extent of DNA replication initiation involved in mitotic DNA replication. Relationships: is a type of negative regulation of DNA-templated DNA replication initiation [GO:0032297]; is a type of negative regulation of mitotic cell cycle DNA replication [GO:1903464]; is a type of regulation of mitotic DNA replication initiation [GO:1903466]; negatively regulates mitotic DNA replication initiation [GO:1902975] Also known as: down regulation of DNA replication initiation involved in mitotic DNA replication, down regulation of DNA replication initiation involved in mitotic cell cycle DNA replication, down-regulation of DNA replication initiation involved in mitotic DNA replication, down-regulation of DNA replication initiation involved in mitotic cell cycle DNA replication, downregulation of DNA replication initiation involved in mitotic DNA replication, downregulation of DNA replication initiation involved in mitotic cell cycle DNA replication, negative regulation of DNA replication initiation involved in mitotic cell cycle DNA replication, inhibition of DNA replication initiation involved in mitotic DNA replication, inhibition of DNA replication initiation involved in mitotic cell cycle DNA replication Subtypes: negative regulation of mitotic DNA replication initiation from late origin [GO:0101018] References: PMID:1234 Sources: GOC:TermGenie, GOC:mtg_cell_cycle, GO_REF:0000058